{
  "term_label": "cytosol",
  "gene": "UniProtKB:Q99759",
  "gene_name": "Mitogen-activated protein kinase kinase kinase 3",
  "term_id": "GO:0005829",
  "gene_symbol": "MAP3K3"
}